{
  "gene": "UniProtKB:Q96M20",
  "term_label": "Unknown cellular component",
  "term_id": "UNKNOWN:0003",
  "gene_name": "Cyclic nucleotide-binding domain-containing protein 2",
  "gene_symbol": "CNBD2"
}